{
  "term_id": "UNKNOWN:0003",
  "gene_name": "Putative methyltransferase-like protein 21E pseudogene",
  "gene": "UniProtKB:A6NDL7",
  "gene_symbol": "METTL21EP",
  "term_label": "Unknown cellular component"
}